{
  "term_id": "GO:0046854",
  "gene_symbol": "PIP5K1C",
  "term_label": "phosphatidylinositol phosphate biosynthetic process",
  "gene": "UniProtKB:O60331",
  "gene_name": "Phosphatidylinositol 4-phosphate 5-kinase type-1 gamma"
}